{
  "gene_name": "Mesothelin-like protein",
  "gene_symbol": "MSLNL",
  "term_id": "GO:0009986",
  "gene": "UniProtKB:Q96KJ4",
  "term_label": "cell surface"
}